{
  "gene_name": "Pyrin and HIN domain-containing protein 1",
  "gene": "UniProtKB:Q6K0P9",
  "term_label": "activation of innate immune response",
  "gene_symbol": "PYHIN1",
  "term_id": "GO:0002218"
}